{
  "term_label": "cytoplasm",
  "gene_name": "Stromal membrane-associated protein 1",
  "term_id": "GO:0005737",
  "gene": "UniProtKB:Q8IYB5",
  "gene_symbol": "SMAP1"
}